{
  "term_id": "GO:0005737",
  "gene": "UniProtKB:O60477",
  "gene_name": "BMP_retinoic acid-inducible neural-specific protein 1",
  "term_label": "cytoplasm",
  "gene_symbol": "BRINP1"
}